heart morphogenesis [GO:0003007] (BP) Definition: The developmental process in which the heart is generated and organized. The heart is a hollow, muscular organ, which, by contracting rhythmically, keeps up the circulation of the blood. Regulation: regulated by regulation of heart morphogenesis [GO:2000826] Relationships: is_a animal organ morphogenesis [GO:0009887]; is part of GO:0007507 Sources: GOC:dph, GOC:isa_complete Also known as: cardiac morphogenesis